{
  "gene_name": "Olfactory receptor 1K1",
  "term_id": "GO:0050911",
  "term_label": "detection of chemical stimulus involved in sensory perception of smell",
  "gene_symbol": "OR1K1",
  "gene": "UniProtKB:Q8NGR3"
}